{
  "gene_symbol": "TRBV7-3",
  "term_id": "GO:0005886",
  "gene_name": "Probable non-functional T cell receptor beta variable 7-3",
  "gene": "UniProtKB:A0A075B6L6",
  "term_label": "plasma membrane"
}